regulation of tetrapyrrole biosynthetic process from glycine and succinyl-CoA [GO:1901413] (biological process) Relationships: is a type of regulation of amino acid metabolic process [GO:0006521]; is a type of regulation of nucleobase-containing compound metabolic process [GO:0019219]; is a type of regulation of amide metabolic process [GO:0034248]; is a type of regulation of sulfur metabolic process [GO:0042762]; is a type of regulation of phosphorus metabolic process [GO:0051174]; is a type of regulation of small molecule metabolic process [GO:0062012]; is a type of regulation of tetrapyrrole biosynthetic process [GO:1901463]; regulates tetrapyrrole biosynthetic process from glycine and succinyl-CoA [GO:0033527] Also known as: regulation of tetrapyrrole anabolism from glycine and succinyl-CoA, regulation of tetrapyrrole biosynthesis from glycine and succinyl-CoA, regulation of tetrapyrrole formation from glycine and succinyl-CoA, regulation of tetrapyrrole synthesis from glycine and succinyl-CoA Subtypes: negative regulation of tetrapyrrole biosynthetic process from glycine and succinyl-CoA [GO:1901414], positive regulation of tetrapyrrole biosynthetic process from glycine and succinyl-CoA [GO:1901415] Sources: GOC:TermGenie, GOC:mengo_curators Definition: Any process that modulates the frequency, rate or extent of tetrapyrrole biosynthetic process from glycine and succinyl-CoA.